{
  "gene_name": "Polypeptide N-acetylgalactosaminyltransferase 12",
  "gene_symbol": "GALNT12",
  "term_label": "Golgi apparatus",
  "gene": "UniProtKB:Q8IXK2",
  "term_id": "GO:0005794"
}